{
  "gene_symbol": "ZNF528",
  "term_id": "GO:0005634",
  "gene_name": "Zinc finger protein 528",
  "gene": "UniProtKB:Q3MIS6",
  "term_label": "nucleus"
}